{
  "term_id": "GO:0006954",
  "gene_symbol": "PTGDR",
  "gene": "UniProtKB:Q13258",
  "gene_name": "Prostaglandin D2 receptor",
  "term_label": "inflammatory response"
}